regulation of octadecene biosynthetic process [GO:1900914] (biological process) Subtypes: negative regulation of octadecene biosynthetic process [GO:1900915], GO:1900916 Relationships: is a type of regulation of olefin biosynthetic process [GO:1900911]; regulates octadecene biosynthetic process [GO:1900682] Definition: Any process that modulates the frequency, rate or extent of octadecene biosynthetic process. Sources: GOC:TermGenie, GOC:mengo_curators Also known as: regulation of 1-octadecene biosynthetic process, regulation of octadecene anabolism, regulation of octadecene biosynthesis, regulation of octadecene formation, regulation of octadecene synthesis